{
  "gene_name": "Homeobox protein OTX2",
  "term_id": "GO:0006357",
  "term_label": "regulation of transcription by RNA polymerase II",
  "gene": "UniProtKB:P32243",
  "gene_symbol": "OTX2"
}